tricoumaroylspermidine meta-hydroxylase activity [GO:0072547] (molecular function) Definition: Catalysis of the reaction: tricoumaroyl spermidine + NADPH + O2 = dicoumaroyl monocaffeoyl spermidine + NADP+ + H2O. Also known as: tricoumaroyl spermidine meta-hydroxylase activity References: PMID:19779199 Sources: GOC:kad Relationships: is a type of tri-(coumaroyl or caffeoyl) spermidine meta-hydroxylase activity [GO:0072533]